response to methionine [GO:1904640] (biological process) Definition: Any process that results in a change in state or activity of a cell or an organism (in terms of movement, secretion, enzyme production, gene expression, etc.) as a result of a methionine stimulus. Subtypes: cellular response to methionine [GO:0061431] Relationships: is a type of response to amino acid [GO:0043200]; is a type of response to nitrogen compound [GO:1901698]; is a type of response to oxygen-containing compound [GO:1901700] References: PMID:17716000 Sources: GOC:TermGenie, GO_REF:0000071